{
  "gene": "UniProtKB:O15504",
  "gene_name": "Nucleoporin NUP42",
  "term_id": "GO:0005049",
  "term_label": "nuclear export signal receptor activity",
  "gene_symbol": "NUP42"
}